{
  "gene": "UniProtKB:Q8TAE7",
  "gene_name": "Potassium voltage-gated channel subfamily G member 3",
  "gene_symbol": "KCNG3",
  "term_id": "GO:0008076",
  "term_label": "voltage-gated potassium channel complex"
}